{
  "term_label": "transcription coactivator activity",
  "gene_symbol": "MED20",
  "gene_name": "Mediator of RNA polymerase II transcription subunit 20",
  "term_id": "GO:0003713",
  "gene": "UniProtKB:Q9H944"
}